positive regulation of lymphotoxin A production [GO:0032761] (biological process) Sources: GOC:mah Relationships: is a type of GO:0032681; is a type of positive regulation of protein metabolic process [GO:0051247]; is a type of positive regulation of tumor necrosis factor superfamily cytokine production [GO:1903557]; positively regulates lymphotoxin A production [GO:0032641] Definition: Any process that activates or increases the frequency, rate, or extent of lymphotoxin A production. Also known as: positive regulation of LTA production, positive regulation of TNF-beta production, positive regulation of lymphotoxin-alpha production, positive regulation of tumor necrosis factor-beta production, up regulation of lymphotoxin A production, up-regulation of lymphotoxin A production, upregulation of lymphotoxin A production, activation of lymphotoxin A production, positive regulation of lymphotoxin A biosynthetic process, stimulation of lymphotoxin A production